{
  "term_label": "G protein-coupled receptor activity",
  "term_id": "GO:0004930",
  "gene": "UniProtKB:Q99680",
  "gene_symbol": "GPR22",
  "gene_name": "G-protein coupled receptor 22"
}